{
  "term_label": "Unknown cellular component",
  "term_id": "UNKNOWN:0003",
  "gene": "UniProtKB:P52747",
  "gene_name": "Zinc finger protein 143",
  "gene_symbol": "ZNF143"
}